{
  "gene_symbol": "ASIC1",
  "term_id": "GO:0005886",
  "term_label": "plasma membrane",
  "gene": "UniProtKB:P78348",
  "gene_name": "Acid-sensing ion channel 1"
}